fungal-type cell wall polysaccharide metabolic process [GO:0071966] (biological process) Definition: The chemical reactions and pathways involving the polysaccharides which make up the fungal-type cell wall. Sources: GOC:mah Subtypes: fungal-type cell wall polysaccharide biosynthetic process [GO:0051278], fungal-type cell wall (1->3)-alpha-glucan metabolic process [GO:0070599], GO:0070879 Relationships: is a type of cell wall polysaccharide metabolic process [GO:0010383]; is part of fungal-type cell wall organization or biogenesis [GO:0071852]